positive regulation of cardiac muscle tissue growth [GO:0055023] (biological process) Also known as: positive regulation of heart muscle growth, up regulation of cardiac muscle growth, up-regulation of cardiac muscle growth, upregulation of cardiac muscle growth, activation of cardiac muscle growth, stimulation of cardiac muscle growth Sources: GOC:vk Definition: Any process that activates, maintains or increases the frequency, rate or extent of cardiac muscle growth. Subtypes: positive regulation of cardiac muscle cell proliferation [GO:0060045], positive regulation of cell growth involved in cardiac muscle cell development [GO:0061051] Relationships: is a type of GO:0055021; is a type of positive regulation of heart growth [GO:0060421]; positively regulates GO:0055017